{
  "gene_name": "FMR1-interacting protein NUFIP2",
  "gene_symbol": "NUFIP2",
  "gene": "UniProtKB:Q7Z417",
  "term_label": "cytoplasmic stress granule",
  "term_id": "GO:0010494"
}